{
  "gene": "UniProtKB:Q9UIG0",
  "gene_symbol": "BAZ1B",
  "term_id": "GO:0090535",
  "term_label": "WICH complex",
  "gene_name": "Tyrosine-protein kinase BAZ1B"
}